{
  "term_id": "UNKNOWN:0003",
  "gene_name": "Nuclear receptor coactivator 4",
  "gene_symbol": "NCOA4",
  "term_label": "Unknown cellular component",
  "gene": "UniProtKB:Q13772"
}